{
  "term_label": "Unknown molecular function",
  "gene_symbol": "CDON",
  "term_id": "UNKNOWN:0001",
  "gene": "UniProtKB:Q4KMG0",
  "gene_name": "Cell adhesion molecule-related_down-regulated by oncogenes"
}